{
  "term_id": "GO:0005634",
  "gene_name": "Axin-1",
  "gene": "UniProtKB:O15169",
  "gene_symbol": "AXIN1",
  "term_label": "nucleus"
}